negative regulation of Schwann cell proliferation [GO:0010626] (biological process) Relationships: is a type of regulation of Schwann cell proliferation [GO:0010624]; is a type of negative regulation of glial cell proliferation [GO:0060253]; negatively regulates Schwann cell proliferation [GO:0014010] Sources: GOC:dph, GOC:sl, GOC:tb Definition: Any process that decreases the frequency or extent of the multiplication or reproduction of Schwann cells, resulting in the expansion of their population. Schwann cells are a type of glial cell in the peripheral nervous system. Subtypes: negative regulation of Schwann cell proliferation involved in axon regeneration [GO:1905045]